{
  "gene_name": "A disintegrin and metalloproteinase with thrombospondin motifs 1",
  "gene": "UniProtKB:Q9UHI8",
  "term_label": "extracellular matrix",
  "gene_symbol": "ADAMTS1",
  "term_id": "GO:0031012"
}